negative regulation of renin secretion into blood stream [GO:1900134] (BP) Relationships: is a type of negative regulation of protein secretion [GO:0050709]; is a type of GO:1900133; negatively regulates renin secretion into blood stream [GO:0002001] Sources: GOC:TermGenie Also known as: down regulation of renin release into blood stream, down regulation of renin secretion into blood stream, down-regulation of renin release into blood stream, down-regulation of renin secretion into blood stream, downregulation of renin release into blood stream, downregulation of renin secretion into blood stream, negative regulation of renin release into blood stream, inhibition of renin release into blood stream, inhibition of renin secretion into blood stream Definition: Any process that stops, prevents or reduces the frequency, rate or extent of renin secretion into blood stream.